{
  "gene_name": "Olfactory receptor 3A3",
  "gene": "UniProtKB:P47888",
  "term_label": "signal transduction",
  "gene_symbol": "OR3A3",
  "term_id": "GO:0007165"
}